{
  "gene": "UniProtKB:Q68DX3",
  "gene_name": "FERM and PDZ domain-containing protein 2",
  "term_id": "GO:0045177",
  "gene_symbol": "FRMPD2",
  "term_label": "apical part of cell"
}